chemokine (C-C motif) ligand 19 binding [GO:0035757] (molecular function) Also known as: CCL19 binding Sources: GOC:BHF Definition: Binding to chemokine (C-C motif) ligand 19. Relationships: is_a GO:0019957